{
  "gene_name": "Zinc finger protein 496",
  "term_id": "GO:0000981",
  "gene_symbol": "ZNF496",
  "term_label": "DNA-binding transcription factor activity, RNA polymerase II-specific",
  "gene": "UniProtKB:Q96IT1"
}